{
  "gene_symbol": "FAM20A",
  "gene": "UniProtKB:Q96MK3",
  "term_label": "enamel mineralization",
  "term_id": "GO:0070166",
  "gene_name": "Pseudokinase FAM20A"
}